spherule viral factory [GO:0039717] (cellular component) Sources: VZ:1951 Relationships: is a type of cytoplasmic viral factory [GO:0039714] Definition: A cytoplasmic viral factory which is a 50-400nm diameter membrane invagination. Spherules can appear on several enveloped cellular components depending on the virus.